{
  "term_label": "multivesicular body",
  "gene_symbol": "CHMP1A",
  "gene_name": "Charged multivesicular body protein 1a",
  "gene": "UniProtKB:Q9HD42",
  "term_id": "GO:0005771"
}